{
  "gene_symbol": "SEMA3C",
  "term_label": "chemorepellent activity",
  "term_id": "GO:0045499",
  "gene": "UniProtKB:Q99985",
  "gene_name": "Semaphorin-3C"
}